{
  "gene": "UniProtKB:Q13190",
  "gene_name": "Syntaxin-5",
  "gene_symbol": "STX5",
  "term_label": "endomembrane system",
  "term_id": "GO:0012505"
}